{
  "term_label": "animal organ development",
  "term_id": "GO:0048513",
  "gene": "UniProtKB:A7XYQ1",
  "gene_name": "Sine oculis-binding protein homolog",
  "gene_symbol": "SOBP"
}